{
  "gene_symbol": "USP17L4",
  "gene": "UniProtKB:A6NCW7",
  "term_label": "cysteine-type deubiquitinase activity",
  "term_id": "GO:0004843",
  "gene_name": "Inactive ubiquitin carboxyl-terminal hydrolase 17-like protein 4"
}